{
  "gene_symbol": "LRRC7",
  "gene": "UniProtKB:Q96NW7",
  "term_label": "establishment or maintenance of epithelial cell apical/basal polarity",
  "gene_name": "Leucine-rich repeat-containing protein 7",
  "term_id": "GO:0045197"
}